negative regulation of aflatoxin biosynthetic process [GO:1900178] (biological process) Relationships: is a type of negative regulation of small molecule metabolic process [GO:0062014]; is a type of regulation of aflatoxin biosynthetic process [GO:1900177]; is a type of negative regulation of secondary metabolite biosynthetic process [GO:1900377]; negatively regulates aflatoxin biosynthetic process [GO:0045122] Also known as: down regulation of aflatoxin anabolism, down regulation of aflatoxin biosynthesis, down regulation of aflatoxin biosynthetic process, down regulation of aflatoxin formation, down regulation of aflatoxin synthesis, down-regulation of aflatoxin anabolism, down-regulation of aflatoxin biosynthesis, down-regulation of aflatoxin biosynthetic process, down-regulation of aflatoxin formation, down-regulation of aflatoxin synthesis, downregulation of aflatoxin anabolism, downregulation of aflatoxin biosynthesis, downregulation of aflatoxin biosynthetic process, downregulation of aflatoxin formation, downregulation of aflatoxin synthesis, negative regulation of aflatoxin anabolism, negative regulation of aflatoxin biosynthesis, negative regulation of aflatoxin formation, negative regulation of aflatoxin synthesis, inhibition of aflatoxin anabolism, inhibition of aflatoxin biosynthesis, inhibition of aflatoxin biosynthetic process, inhibition of aflatoxin formation, inhibition of aflatoxin synthesis Sources: GOC:di Definition: Any process that stops, prevents or reduces the frequency, rate or extent of aflatoxin biosynthetic process.